{
  "gene_name": "Creatine kinase B-type",
  "gene": "UniProtKB:P12277",
  "gene_symbol": "CKB",
  "term_label": "phosphocreatine biosynthetic process",
  "term_id": "GO:0046314"
}